VEGF-activated platelet-derived growth factor receptor-alpha signaling pathway [GO:0038087] (biological process) Definition: The series of molecular signals initiated by vascular endothelial growth factor (VEGF) binding to an alpha-type platelet-derived growth factor receptor (PDGFR) on the surface of a cell, and ending with the regulation of a downstream cellular process, e.g. transcription. References: PMID:17470632 Sources: GOC:signaling Relationships: is a type of platelet-derived growth factor receptor-alpha signaling pathway [GO:0035790]; is a type of GO:0038086 Also known as: VEGF-activated PDGFRalpha signalling pathway, VEGF-activated platelet-derived growth factor receptor-alpha signalling pathway, VEGF/PDGFRalpha signaling pathway, vascular endothelial growth factor-activated platelet-derived growth factor receptor-alpha signaling pathway, VEGF-A/PDGFRalpha signaling